{
  "gene": "UniProtKB:Q6UWY2",
  "term_id": "GO:0005615",
  "gene_name": "Serine protease 57",
  "gene_symbol": "PRSS57",
  "term_label": "extracellular space"
}